{
  "gene_symbol": "NR1H4",
  "gene_name": "Bile acid receptor",
  "term_label": "negative regulation of transcription by RNA polymerase II",
  "gene": "UniProtKB:Q96RI1",
  "term_id": "GO:0000122"
}